{
  "term_label": "Unknown molecular function",
  "gene": "UniProtKB:Q15543",
  "term_id": "UNKNOWN:0001",
  "gene_name": "Transcription initiation factor TFIID subunit 13",
  "gene_symbol": "TAF13"
}